host cell plastid [GO:0033651] (cellular component) Definition: Any member of a family of organelles as found in the cytoplasm of host cells, which are membrane-bounded and contain DNA. The host is defined as the larger of the organisms involved in a symbiotic interaction. Sources: GOC:pamgo_curators Relationships: is a type of host intracellular membrane-bounded organelle [GO:0033648] Subtypes: host cell chloroplast [GO:0033652]